negative regulation of late stripe melanocyte differentiation [GO:0050949] (biological process) Definition: Any process that stops, prevents, or reduces the frequency, rate or extent of late stripe melanocyte differentiation. Sources: GOC:ai Also known as: down regulation of late stripe melanocyte differentiation, down-regulation of late stripe melanocyte differentiation, downregulation of late stripe melanocyte differentiation, negative regulation of late stripe melanophore differentiation, inhibition of late stripe melanocyte differentiation Relationships: is_a negative regulation of melanocyte differentiation [GO:0045635]; is_a regulation of late stripe melanocyte differentiation [GO:0050940]; negatively regulates GO:0050934